{
  "term_label": "synapse organization",
  "term_id": "GO:0050808",
  "gene_symbol": "CNTN6",
  "gene": "UniProtKB:Q9UQ52",
  "gene_name": "Contactin-6"
}